{
  "term_label": "GTPase activity",
  "gene_name": "Ras-related protein R-Ras",
  "term_id": "GO:0003924",
  "gene_symbol": "RRAS",
  "gene": "UniProtKB:P10301"
}